box C/D sno(s)RNA processing [GO:0034963] (biological process) Subtypes: box C/D sno(s)RNA 3'-end processing [GO:0000494], GO:0034965, box C/D sno(s)RNA 5'-end processing [GO:0106410] Definition: Any process involved in the conversion of a primary box C/D type small RNA transcript into a mature box C/D RNA. Relationships: is a type of GO:0033967; is a type of GO:0043144 Also known as: box C/D sRNA processing, box C/D snoRNA processing Sources: GOC:krc, GOC:mah